{
  "gene_symbol": "RNASE2",
  "gene_name": "Non-secretory ribonuclease",
  "gene": "UniProtKB:P10153",
  "term_id": "GO:0002227",
  "term_label": "innate immune response in mucosa"
}